autophagosome maturation [GO:0097352] (biological process) Definition: Removal of PI3P and Atg8/LC3 after the closure of the phagophore and before the fusion with the endosome/lysosome (e.g. mammals and insects) or vacuole (yeast), and that very likely destabilizes other Atg proteins and thus enables their efficient dissociation and recycling. References: PMID:28077293 Sources: GOC:autophagy, GOC:lf Also known as: autophagic vacuole fusion, autophagic vacuole maturation, autophagosome fusion Relationships: is_a protein-containing complex disassembly [GO:0032984]; is part of macroautophagy [GO:0016236] Regulation: RO_0002211 by GO:1901096; RO_0002212 by GO:1901097; positively regulated by positive regulation of autophagosome maturation [GO:1901098]